{
  "gene_symbol": "ATCAY",
  "gene_name": "Caytaxin",
  "term_label": "Unknown molecular function",
  "term_id": "UNKNOWN:0001",
  "gene": "UniProtKB:Q86WG3"
}